mRNA cleavage factor complex [GO:0005849] (cellular component) Subtypes: GO:0005847, mRNA cleavage stimulating factor complex [GO:0005848] Relationships: is a type of nuclear protein-containing complex [GO:0140513] References: PMID:10357856 Sources: GOC:mah Definition: Any macromolecular complex involved in cleavage or polyadenylation of mRNA molecules.